{
  "gene": "UniProtKB:Q5TCH4",
  "term_id": "GO:0019369",
  "term_label": "arachidonate metabolic process",
  "gene_symbol": "CYP4A22",
  "gene_name": "Cytochrome P450 4A22"
}